rhamnose:proton symporter activity [GO:0015561] (molecular function) Definition: Enables the transfer of a solute or solutes from one side of a membrane to the other according to the reaction: rhamnose(out) + H+(out) = rhamnose(in) + H+(in). Relationships: is a type of GO:0009679; is a type of GO:0015153 Sources: TC:2.A.7.6 Also known as: rhamnose:hydrogen symporter activity